{
  "gene_name": "Phosphatidylinositol 3,4,5-trisphosphate-dependent Rac exchanger 1 protein",
  "gene_symbol": "PREX1",
  "gene": "UniProtKB:Q8TCU6",
  "term_label": "plasma membrane",
  "term_id": "GO:0005886"
}